{
  "gene": "UniProtKB:Q9NQ39",
  "term_label": "structural constituent of ribosome",
  "gene_symbol": "RPS10P5",
  "term_id": "GO:0003735",
  "gene_name": "Putative ribosomal protein eS10-like"
}